{
  "term_id": "GO:0046975",
  "gene_symbol": "SETD4",
  "gene": "UniProtKB:Q9NVD3",
  "gene_name": "SET domain-containing protein 4",
  "term_label": "histone H3K36 methyltransferase activity"
}